{
  "gene_name": "Syntaphilin",
  "term_id": "GO:0030182",
  "gene_symbol": "SNPH",
  "term_label": "neuron differentiation",
  "gene": "UniProtKB:O15079"
}